{
  "gene_name": "Nuclear transcription factor Y subunit alpha",
  "term_id": "GO:0016602",
  "gene_symbol": "NFYA",
  "term_label": "CCAAT-binding factor complex",
  "gene": "UniProtKB:P23511"
}